cleavage furrow leading edge [GO:0090689] (cellular component) Definition: The 'trough' of the cleavage furrow. This is the part of the cleavage furrow closest to the contractile ring. References: PMID:27082518 Sources: GOC:vw Relationships: is a type of GO:0110165; is part of cleavage furrow [GO:0032154]